{
  "gene": "UniProtKB:Q9GZN6",
  "gene_name": "Orphan sodium- and chloride-dependent neurotransmitter transporter NTT5",
  "gene_symbol": "SLC6A16",
  "term_label": "sodium ion transmembrane transport",
  "term_id": "GO:0035725"
}